{
  "term_id": "UNKNOWN:0003",
  "gene_name": "NACHT and WD repeat domain-containing protein 2",
  "term_label": "Unknown cellular component",
  "gene": "UniProtKB:Q9ULI1",
  "gene_symbol": "NWD2"
}